vagus nerve structural organization [GO:0021645] (biological process) Definition: The process that contributes to the act of creating the structural organization of the vagus nerve. This process pertains to the physical shaping of a rudimentary structure. This nerve is primarily sensory but also has visceromotor components. It originates in the brain stem and controls many autonomic functions of the heart, lungs, stomach, pharynx, larynx, trachea, esophagus and other gastrointestinal tract components. It controls some motor functions such as speech. The sensory branches mediate sensation from the pharynx, larynx, thorax and abdomen; it also innervates taste buds in the epiglottis. Sources: GOC:cls, GOC:dgh, GOC:dph, GOC:jid, GO_REF:0000021 Also known as: vagus nerve structural organisation, CN X structural organization Relationships: is a type of cranial nerve structural organization [GO:0021604]; is part of vagus nerve morphogenesis [GO:0021644]